meiotic spindle organization [GO:0000212] (biological process) Subtypes: meiotic spindle disassembly [GO:0051229], meiotic spindle assembly [GO:0090306] Also known as: meiotic spindle organisation, spindle organization during meiosis, meiotic spindle organization and biogenesis, meiotic spindle stabilization Definition: A process that is carried out at the cellular level which results in the assembly, arrangement of constituent parts, or disassembly of the microtubule spindle during a meiotic cell cycle. Sources: GOC:go_curators, GOC:mah Relationships: is a type of spindle organization [GO:0007051]; is a type of meiotic cell cycle process [GO:1903046]